{
  "gene_symbol": "COX6A1",
  "term_id": "GO:0006123",
  "term_label": "mitochondrial electron transport, cytochrome c to oxygen",
  "gene": "UniProtKB:P12074",
  "gene_name": "Cytochrome c oxidase subunit 6A1, mitochondrial"
}